{
  "gene": "UniProtKB:Q8N682",
  "term_id": "UNKNOWN:0001",
  "term_label": "Unknown molecular function",
  "gene_name": "DNA damage-regulated autophagy modulator protein 1",
  "gene_symbol": "DRAM1"
}